{
  "gene_symbol": "SPRED2",
  "term_id": "GO:0070373",
  "term_label": "negative regulation of ERK1 and ERK2 cascade",
  "gene_name": "Sprouty-related, EVH1 domain-containing protein 2",
  "gene": "UniProtKB:Q7Z698"
}